ERK1 and ERK2 cascade [GO:0070371] (biological process) References: PMID:20811974, PMID:23125017, PMID:28903453 Relationships: is_a MAPK cascade [GO:0000165] Also known as: ERK cascade, ERK1 and ERK2 signaling pathway, ERK1 and ERK2 signalling pathway, ERK1/2 cascade, extracellular signal-regulated kinase 1/2 (ERK1/2) cascade, extracellular signal-regulated kinase 1/2 cascade, ERK1 cascade, ERK2 cascade, MAPK1 cascade, MAPK3 cascade Definition: A MAPK cascade containing at least the ERK1 or ERK2 MAP kinases. It starts with the activation of a MAP3K, and the consecutive activation of a MPK2K and of ERK1 or ERK2. The cascade can also contain an additional tier: the upstream MAP4K. The kinases in each tier phosphorylate and activate the kinase in the downstream tier. The ERK1/ERK2 cascade is activated by mitogens, growth factors, G protein-coupled receptors, and results in cellular responses such as cell proliferation, cell differentiation and development. Regulation: regulated by regulation of ERK1 and ERK2 cascade [GO:0070372]; negatively regulated by negative regulation of ERK1 and ERK2 cascade [GO:0070373]; positively regulated by positive regulation of ERK1 and ERK2 cascade [GO:0070374] Note: Note that this MAPKKK cascade is commonly referred to as the ERK pathway in the literature, but involves only ERK1 or ERK2 and should not be confused with cascades that involve other ERK kinases.